phytosphingosine biosynthetic process [GO:0071602] (biological process) Also known as: phytosphingosine anabolism, phytosphingosine biosynthesis, phytosphingosine formation, phytosphingosine synthesis Definition: The chemical reactions and pathways resulting in the formation of phytosphingosine, (2S,3S,4R)-2-aminooctadecane-1,3,4-triol. Sources: GOC:mah Relationships: is a type of GO:0006671; is_a polyol biosynthetic process [GO:0046173]; is a type of GO:0046520